pyrimidine nucleoside diphosphate catabolic process [GO:0009140] (biological process) Subtypes: pyrimidine ribonucleoside diphosphate catabolic process [GO:0009195], pyrimidine deoxyribonucleoside diphosphate catabolic process [GO:0009198] Also known as: pyrimidine nucleoside diphosphate breakdown, pyrimidine nucleoside diphosphate catabolism, pyrimidine nucleoside diphosphate degradation Relationships: is a type of GO:0009134; is a type of GO:0009138 Definition: The chemical reactions and pathways resulting in the breakdown of pyrimidine nucleoside diphosphate, a compound consisting of a pyrimidine base linked to a ribose or deoxyribose sugar esterified with diphosphate on the sugar. Sources: GOC:go_curators, ISBN:0198506732